{
  "term_id": "UNKNOWN:0003",
  "gene": "UniProtKB:Q8NEE8",
  "gene_name": "Tetratricopeptide repeat protein 16",
  "term_label": "Unknown cellular component",
  "gene_symbol": "TTC16"
}